{
  "gene_name": "Phospholipid phosphatase 3",
  "gene": "UniProtKB:O14495",
  "term_label": "phosphatidate phosphatase activity",
  "gene_symbol": "PLPP3",
  "term_id": "GO:0008195"
}